{
  "gene_name": "Retinoic acid receptor gamma",
  "term_label": "negative regulation of transcription by RNA polymerase II",
  "term_id": "GO:0000122",
  "gene": "UniProtKB:P13631",
  "gene_symbol": "RARG"
}